{
  "gene_symbol": "LZTS2",
  "gene_name": "Leucine zipper putative tumor suppressor 2",
  "term_label": "negative regulation of canonical Wnt signaling pathway",
  "term_id": "GO:0090090",
  "gene": "UniProtKB:Q9BRK4"
}